{
  "gene_symbol": "SLC12A6",
  "term_label": "potassium:chloride symporter activity",
  "gene_name": "Solute carrier family 12 member 6",
  "gene": "UniProtKB:Q9UHW9",
  "term_id": "GO:0015379"
}